osteoclast development [GO:0036035] (biological process) Regulation: regulated by regulation of osteoclast development [GO:2001204]; negatively regulated by negative regulation of osteoclast development [GO:2001205]; positively regulated by GO:2001206 Also known as: osteoclast cell development Relationships: is a type of myeloid cell development [GO:0061515]; is a type of bone cell development [GO:0098751]; BFO_0000050 osteoclast differentiation [GO:0030316] Definition: The process whose specific outcome is the progression of a osteoclast from its formation to the mature structure. Cell development does not include the steps involved in committing a cell to a specific fate. An osteoclast is a specialized phagocytic cell associated with the absorption and removal of the mineralized matrix of bone tissue. Sources: CL:0000092, GOC:bf, GOC:yaf